phagophore [GO:0061908] (cellular component) Relationships: is a type of cellular anatomical structure [GO:0110165]; is part of cytoplasm [GO:0005737] Definition: A disk-like structure that expands, rounds up into a cup-shaped structure, and eventually closes around its cargo (for example cytoplasmic components) to become an autophagosome or Cvt vesicle. Also known as: isolation membrane References: PMID:22664348, PMID:24201109